{
  "term_label": "glucose-6-phosphatase activity",
  "gene_name": "Glucose-6-phosphatase 3",
  "gene": "UniProtKB:Q9BUM1",
  "gene_symbol": "G6PC3",
  "term_id": "GO:0004346"
}